{
  "term_id": "GO:0005801",
  "gene_name": "Golgin subfamily A member 6A",
  "gene_symbol": "GOLGA6A",
  "gene": "UniProtKB:Q9NYA3",
  "term_label": "cis-Golgi network"
}